arsenate ion transmembrane transporter activity [GO:1901683] (molecular function) Subtypes: ATPase-coupled arsenite transmembrane transporter activity [GO:0015446] Sources: GOC:TermGenie Definition: Enables the transfer of an arsenate ion from one side of a membrane to the other. Relationships: is a type of transmembrane transporter activity [GO:0022857]; is part of arsenate ion transmembrane transport [GO:1901684]